{
  "gene_symbol": "ARID1B",
  "gene": "UniProtKB:Q8NFD5",
  "term_id": "GO:0016514",
  "gene_name": "AT-rich interactive domain-containing protein 1B",
  "term_label": "SWI/SNF complex"
}